{
  "term_label": "nuclear import signal receptor activity",
  "gene_symbol": "KPNA5",
  "gene": "UniProtKB:O15131",
  "gene_name": "Importin subunit alpha-6",
  "term_id": "GO:0061608"
}